host cell nucleus [GO:0042025] (cellular component) Definition: A membrane-bounded organelle as it is found in the host cell in which chromosomes are housed and replicated. The host is defined as the larger of the organisms involved in a symbiotic interaction. Sources: GOC:pamgo_curators Relationships: is a type of host intracellular membrane-bounded organelle [GO:0033648]